{
  "gene_symbol": "IGLV1-51",
  "term_label": "Unknown molecular function",
  "gene": "UniProtKB:P01701",
  "gene_name": "Immunoglobulin lambda variable 1-51",
  "term_id": "UNKNOWN:0001"
}